{
  "term_id": "GO:0141156",
  "gene": "UniProtKB:P16220",
  "gene_name": "Cyclic AMP-responsive element-binding protein 1",
  "gene_symbol": "CREB1",
  "term_label": "cAMP/PKA signal transduction"
}